low-affinity nitrate transmembrane transporter activity [GO:0080054] (MF) Relationships: is a type of GO:0015112 Also known as: low affinity nitrate transmembrane transporter activity Definition: Enables the transfer of nitrate ions (NO3-) from one side of a membrane to the other. In low-affinity transport the transporter is able to bind the solute only if it is present at very high concentrations. References: PMID:19050168